{
  "gene_symbol": "DPYD",
  "gene_name": "Dihydropyrimidine dehydrogenase [NADP(+)]",
  "gene": "UniProtKB:Q12882",
  "term_id": "GO:0002058",
  "term_label": "uracil binding"
}